{
  "gene": "UniProtKB:Q969J5",
  "term_id": "GO:0019221",
  "gene_symbol": "IL22RA2",
  "gene_name": "Interleukin-22 receptor subunit alpha-2",
  "term_label": "cytokine-mediated signaling pathway"
}